{
  "gene_name": "Olfactory receptor 7D2",
  "term_label": "signal transduction",
  "term_id": "GO:0007165",
  "gene_symbol": "OR7D2",
  "gene": "UniProtKB:Q96RA2"
}